{
  "gene_name": "Killer cell lectin-like receptor subfamily F member 2",
  "gene_symbol": "KLRF2",
  "term_label": "Unknown molecular function",
  "term_id": "UNKNOWN:0001",
  "gene": "UniProtKB:D3W0D1"
}